macromolecule catabolic process [GO:0009057] (biological process) Relationships: is a type of catabolic process [GO:0009056]; is a type of GO:0043170 Also known as: biopolymer catabolic process, macromolecule breakdown, macromolecule catabolism, macromolecule degradation, multicellular organismal macromolecule catabolic process, cellular macromolecule catabolic process, cellular macromolecule catabolism, cellular macromolecule degradation Definition: The chemical reactions and pathways resulting in the breakdown of a macromolecule, any molecule of high relative molecular mass, the structure of which essentially comprises the multiple repetition of units derived, actually or conceptually, from molecules of low relative molecular mass. Sources: GOC:mah Subtypes: GO:0000272, aminoglycan catabolic process [GO:0006026], lipopolysaccharide catabolic process [GO:0009104], cell wall macromolecule catabolic process [GO:0016998], protein catabolic process [GO:0030163], receptor catabolic process [GO:0032801], modification-dependent macromolecule catabolic process [GO:0043632], teichoic acid catabolic process [GO:0070393], GO:0141188, amylopectin catabolic process [GO:2000897]